{
  "gene_name": "Kinesin-like protein KIF24",
  "term_label": "microtubule",
  "gene_symbol": "KIF24",
  "gene": "UniProtKB:Q5T7B8",
  "term_id": "GO:0005874"
}